{
  "gene_name": "Ankyrin repeat and SOCS box protein 5",
  "term_id": "UNKNOWN:0001",
  "gene_symbol": "ASB5",
  "term_label": "Unknown molecular function",
  "gene": "UniProtKB:Q8WWX0"
}